{
  "term_id": "GO:0005886",
  "gene_symbol": "EPHB3",
  "gene_name": "Ephrin type-B receptor 3",
  "term_label": "plasma membrane",
  "gene": "UniProtKB:P54753"
}